cyclic-di-GMP binding [GO:0035438] (molecular function) Definition: Binding to cyclic-di-GMP, cyclic dimeric guanosine monophosphate. Relationships: is a type of cyclic nucleotide binding [GO:0030551]; is a type of guanyl ribonucleotide binding [GO:0032561]; is a type of anion binding [GO:0043168] Also known as: 3',5'-cyclic di-GMP binding, c-di-GMP binding, cyclic dinucleotide di-GMP binding Sources: GOC:bf